{
  "term_id": "GO:0000981",
  "gene": "UniProtKB:Q15935",
  "gene_symbol": "ZNF77",
  "gene_name": "Zinc finger protein 77",
  "term_label": "DNA-binding transcription factor activity, RNA polymerase II-specific"
}